chemorepulsion of branchiomotor neuron axon in neural tube [GO:0021787] (biological process) Relationships: is a type of branchiomotor neuron axon guidance in neural tube [GO:0021786]; is a type of chemorepulsion of branchiomotor axon [GO:0021793] Also known as: negative chemotaxis of branchiomotor neuron axon in neural tube Definition: The process in which a branchiomotor neuron growth cone in the neural tube is directed to a specific target site in the neural tube in response to a repulsive chemical cue. Branchiomotor neurons are located in the hindbrain and innervate branchial arch-derived muscles that control jaw movements, facial expression, the larynx, and the pharynx. References: PMID:14699587 Sources: GOC:cls, GOC:dgh, GOC:dph, GOC:jid, GO_REF:0000021